{
  "gene_symbol": "PTMS",
  "term_id": "GO:0043066",
  "gene": "UniProtKB:P20962",
  "term_label": "negative regulation of apoptotic process",
  "gene_name": "Parathymosin"
}